{
  "term_label": "proteasome-mediated ubiquitin-dependent protein catabolic process",
  "gene_symbol": "TRIM72",
  "term_id": "GO:0043161",
  "gene": "UniProtKB:Q6ZMU5",
  "gene_name": "Tripartite motif-containing protein 72"
}